{
  "term_label": "immune response",
  "gene_name": "Interleukin-36 receptor antagonist protein",
  "gene_symbol": "IL36RN",
  "gene": "UniProtKB:Q9UBH0",
  "term_id": "GO:0006955"
}